{
  "gene": "UniProtKB:Q9BYG4",
  "term_id": "GO:0005634",
  "term_label": "nucleus",
  "gene_name": "Partitioning defective 6 homolog gamma",
  "gene_symbol": "PARD6G"
}